serine/threonine protein kinase complex [GO:1902554] (cellular component) References: PMID:18191223 Sources: GOC:TermGenie, GOC:bhm Relationships: is a type of protein kinase complex [GO:1902911] Definition: A protein complex which is capable of protein serine/threonine kinase activity. Also known as: PDR16 complex dimer, PDR16 complex homodimer Subtypes: cyclin-dependent protein kinase holoenzyme complex [GO:0000307], cAMP-dependent protein kinase complex [GO:0005952], protein kinase CK2 complex [GO:0005956], GO:0005964, IkappaB kinase complex [GO:0008385], protein kinase 5 complex [GO:0016533], Dbf4-dependent protein kinase complex [GO:0031431], carboxy-terminal domain protein kinase complex [GO:0032806], GO:0034977, activin receptor complex [GO:0048179], transforming growth factor beta ligand-receptor complex [GO:0070021], DNA-dependent protein kinase complex [GO:0070418], PAR polarity complex [GO:0120157], Atg1/ULK1 kinase complex [GO:1990316], Gin4 complex [GO:1990317], GO:1990332, DAPK1-calmodulin complex [GO:1990722] Note: An example is IRE1 in S. cerevisiae (UniProt ID P32361) in PMID:18191223 (inferred from direct assay).